{
  "gene_symbol": "STK4",
  "term_id": "GO:0090090",
  "term_label": "negative regulation of canonical Wnt signaling pathway",
  "gene_name": "Serine_threonine-protein kinase 4",
  "gene": "UniProtKB:Q13043"
}